{
  "gene": "UniProtKB:Q16531",
  "term_label": "Unknown molecular function",
  "gene_symbol": "DDB1",
  "gene_name": "DNA damage-binding protein 1",
  "term_id": "UNKNOWN:0001"
}